{
  "term_id": "UNKNOWN:0002",
  "gene_name": "RING finger protein 224",
  "gene_symbol": "RNF224",
  "gene": "UniProtKB:P0DH78",
  "term_label": "Unknown biological process"
}